{
  "gene_name": "Xin actin-binding repeat-containing protein 2",
  "term_label": "stress fiber",
  "gene": "UniProtKB:A4UGR9",
  "gene_symbol": "XIRP2",
  "term_id": "GO:0001725"
}